pyrimidine nucleoside diphosphate metabolic process [GO:0009138] (biological process) Definition: The chemical reactions and pathways involving pyrimidine nucleoside diphosphate, a compound consisting of a pyrimidine base linked to a ribose or deoxyribose sugar esterified with diphosphate on the sugar. Relationships: is a type of GO:0009132 Subtypes: pyrimidine nucleoside diphosphate biosynthetic process [GO:0009139], pyrimidine nucleoside diphosphate catabolic process [GO:0009140], GO:0009193, pyrimidine deoxyribonucleoside diphosphate metabolic process [GO:0009196] Also known as: pyrimidine nucleoside diphosphate metabolism Sources: GOC:go_curators, ISBN:0198506732